{
  "gene_symbol": "FAM74A6",
  "gene_name": "Protein FAM74A4_A6",
  "term_label": "Unknown cellular component",
  "gene": "UniProtKB:Q5TZK3",
  "term_id": "UNKNOWN:0003"
}